{
  "gene": "UniProtKB:Q0VDF9",
  "term_id": "GO:0005886",
  "term_label": "plasma membrane",
  "gene_name": "Heat shock 70 kDa protein 14",
  "gene_symbol": "HSPA14"
}